{
  "gene_name": "Cysteine and glycine-rich protein 1",
  "term_label": "Z disc",
  "term_id": "GO:0030018",
  "gene_symbol": "CSRP1",
  "gene": "UniProtKB:P21291"
}